{
  "term_id": "GO:0006357",
  "term_label": "regulation of transcription by RNA polymerase II",
  "gene_symbol": "ZIC4",
  "gene_name": "Zinc finger protein ZIC 4",
  "gene": "UniProtKB:Q8N9L1"
}